DNA (cytosine-5-)-methyltransferase activity, acting on CpN substrates [GO:0051719] (molecular function) Relationships: is a type of GO:0003886 Definition: Catalysis of the reaction: S-adenosyl-L-methionine + DNA containing CpN = S-adenosyl-L-homocysteine + DNA containing 5-MeCpN. References: PMID:15689527